{
  "gene": "UniProtKB:Q8N6L1",
  "term_id": "UNKNOWN:0001",
  "gene_symbol": "KRTCAP2",
  "term_label": "Unknown molecular function",
  "gene_name": "Keratinocyte-associated protein 2"
}